{
  "gene_symbol": "ATG2A",
  "gene": "UniProtKB:Q2TAZ0",
  "gene_name": "Autophagy-related protein 2 homolog A",
  "term_label": "glycophagy",
  "term_id": "GO:0061723"
}